{
  "gene_symbol": "PCGF6",
  "gene_name": "Polycomb group RING finger protein 6",
  "term_id": "GO:0006357",
  "gene": "UniProtKB:Q9BYE7",
  "term_label": "regulation of transcription by RNA polymerase II"
}